{
  "gene": "UniProtKB:O75925",
  "term_label": "chromatin",
  "gene_symbol": "PIAS1",
  "gene_name": "E3 SUMO-protein ligase PIAS1",
  "term_id": "GO:0000785"
}